{
  "term_id": "GO:0005634",
  "term_label": "nucleus",
  "gene_name": "Zinc finger protein 80",
  "gene": "UniProtKB:P51504",
  "gene_symbol": "ZNF80"
}